pectin lyase activity [GO:0047490] (molecular function) Relationships: is a type of carbon-oxygen lyase activity, acting on polysaccharides [GO:0016837] Sources: EC:4.2.2.10 Also known as: pectin trans-eliminase activity, (1->4)-6-O-methyl-alpha-D-galacturonan lyase activity, PL activity, PMGL activity, PNL activity, endo-pectin lyase activity, pectin methyltranseliminase activity, pectolyase activity, polymethylgalacturonic transeliminase activity Definition: Catalysis of the reaction: a pectin = an oligosaccharide with 4-deoxy-6-O-methyl-alpha-D-galact-4-enuronate end + a pectin. This reaction is the eliminative cleavage of (1->4)-alpha-D-galacturonan methyl ester to give oligosaccharides with 4-deoxy-6-O-methyl-alpha-D-galact-4-enuronosyl groups at their nonreducing ends.